{
  "term_label": "intermediate filament organization",
  "gene": "UniProtKB:P35527",
  "gene_name": "Keratin, type I cytoskeletal 9",
  "gene_symbol": "KRT9",
  "term_id": "GO:0045109"
}